{
  "term_label": "Unknown cellular component",
  "gene": "UniProtKB:Q86T20",
  "gene_name": "Small integral membrane protein 29",
  "term_id": "UNKNOWN:0003",
  "gene_symbol": "SMIM29"
}